{
  "term_label": "plasma membrane",
  "gene_symbol": "CLDN6",
  "gene_name": "Claudin-6",
  "term_id": "GO:0005886",
  "gene": "UniProtKB:P56747"
}